positive regulation of leukocyte activation [GO:0002696] (biological process) Sources: GOC:add Relationships: is a type of positive regulation of immune system process [GO:0002684]; is a type of regulation of leukocyte activation [GO:0002694]; is a type of positive regulation of cell activation [GO:0050867]; positively regulates leukocyte activation [GO:0045321] Subtypes: positive regulation of myeloid dendritic cell activation [GO:0030887], GO:0033005, positive regulation of macrophage activation [GO:0043032], GO:0051251, GO:1902565, positive regulation of eosinophil activation [GO:1902568] Definition: Any process that activates or increases the frequency, rate, or extent of leukocyte activation. Also known as: positive regulation of immune cell activation, positive regulation of leucocyte activation, up regulation of leukocyte activation, up-regulation of leukocyte activation, upregulation of leukocyte activation, activation of leukocyte activation, stimulation of leukocyte activation